{
  "term_id": "GO:0008236",
  "term_label": "serine-type peptidase activity",
  "gene": "UniProtKB:O60235",
  "gene_name": "Transmembrane protease serine 11D",
  "gene_symbol": "TMPRSS11D"
}